{
  "term_label": "Golgi apparatus",
  "term_id": "GO:0005794",
  "gene": "UniProtKB:Q5JT25",
  "gene_symbol": "RAB41",
  "gene_name": "Ras-related protein Rab-41"
}